{
  "gene_symbol": "ETF1",
  "term_id": "GO:0005829",
  "gene_name": "Eukaryotic peptide chain release factor subunit 1",
  "gene": "UniProtKB:P62495",
  "term_label": "cytosol"
}